UAC codon-amino acid adaptor activity [GO:0033410] (molecular function) Definition: A triplet codon-amino acid adaptor activity that recognizes a UAC codon. Sources: GOC:mah Relationships: is a type of triplet codon-amino acid adaptor activity [GO:0030533] Note: Note that in the standard genetic code, TAC codes for tyrosine. Also known as: TAC codon-amino acid adaptor activity, tyrosine tRNA